negative regulation of neuron remodeling [GO:1904800] (biological process) Relationships: is a type of negative regulation of neuron maturation [GO:0014043]; is a type of GO:1904799; negatively regulates neuron remodeling [GO:0016322] Also known as: down regulation of neuron remodeling, down regulation of neuronal remodeling, down-regulation of neuron remodeling, down-regulation of neuronal remodeling, downregulation of neuron remodeling, downregulation of neuronal remodeling, negative regulation of neuron remodelling, negative regulation of neuronal remodeling, down regulation of axon pruning, down-regulation of axon pruning, downregulation of axon pruning, inhibition of axon pruning, inhibition of neuron remodeling, inhibition of neuronal remodeling, negative regulation of axon pruning Note: cyy-1 in C. Elegans (P34624) in PMID:21609829 (inferred from mutant phenotype) References: PMID:21609829 Sources: GOC:TermGenie, GO_REF:0000058 Definition: Any process that stops, prevents or reduces the frequency, rate or extent of neuron remodeling.